{
  "term_label": "apoptotic process",
  "gene_symbol": "CASP10",
  "term_id": "GO:0006915",
  "gene": "UniProtKB:Q92851",
  "gene_name": "Caspase-10"
}